{
  "term_id": "GO:0006357",
  "term_label": "regulation of transcription by RNA polymerase II",
  "gene_name": "Zinc finger protein 527",
  "gene": "UniProtKB:Q8NB42",
  "gene_symbol": "ZNF527"
}